regulation of transcription by glucose [GO:0046015] (biological process) Subtypes: regulation of transcription from RNA polymerase II promoter by glucose [GO:0000430], GO:0046016, negative regulation of transcription by glucose [GO:0061986] Relationships: is_a regulation of DNA-templated transcription [GO:0006355] Sources: GOC:go_curators Definition: Any process involving glucose that modulates the frequency, rate or extent or transcription.